{
  "term_id": "GO:0006357",
  "gene_symbol": "RFX3",
  "term_label": "regulation of transcription by RNA polymerase II",
  "gene_name": "Transcription factor RFX3",
  "gene": "UniProtKB:P48380"
}